{
  "term_label": "epithelial cell differentiation",
  "gene": "UniProtKB:Q6A163",
  "term_id": "GO:0030855",
  "gene_name": "Keratin, type I cytoskeletal 39",
  "gene_symbol": "KRT39"
}